{
  "gene_name": "Ras-related GTP-binding protein B",
  "gene_symbol": "RRAGB",
  "gene": "UniProtKB:Q5VZM2",
  "term_id": "GO:0003924",
  "term_label": "GTPase activity"
}